cysteine-type endopeptidase activator activity involved in apoptotic process [GO:0008656] (molecular function) Note: Examples of this are 1) granzymes that may bind to initiator caspases and cleave them, and 2) already active caspases, e.g. caspase 9, that cleave effector caspases. Also known as: caspase activator activity Definition: Binds to and increases the rate of proteolysis catalyzed by a cysteine-type endopeptidase involved in the apoptotic process. Sources: GOC:mah, GOC:mtg_apoptosis Relationships: is a type of peptidase activator activity involved in apoptotic process [GO:0016505]; is_a cysteine-type endopeptidase regulator activity involved in apoptotic process [GO:0043028]